{
  "gene_symbol": "FERMT2",
  "term_label": "focal adhesion",
  "gene": "UniProtKB:Q96AC1",
  "term_id": "GO:0005925",
  "gene_name": "Fermitin family homolog 2"
}